{
  "term_label": "GPI anchor biosynthetic process",
  "gene": "UniProtKB:Q9H720",
  "gene_name": "PGAP2-interacting protein",
  "gene_symbol": "CWH43",
  "term_id": "GO:0006506"
}